{
  "gene": "UniProtKB:Q96L94",
  "term_label": "phosphatidylinositol phosphate binding",
  "gene_symbol": "SNX22",
  "term_id": "GO:1901981",
  "gene_name": "Sorting nexin-22"
}